{
  "gene_symbol": "EIF3A",
  "gene": "UniProtKB:Q14152",
  "term_label": "formation of cytoplasmic translation initiation complex",
  "term_id": "GO:0001732",
  "gene_name": "Eukaryotic translation initiation factor 3 subunit A"
}